{
  "gene": "UniProtKB:P02812",
  "gene_name": "Basic salivary proline-rich protein 2",
  "gene_symbol": "PRB2",
  "term_id": "UNKNOWN:0003",
  "term_label": "Unknown cellular component"
}